{
  "gene_name": "THO complex subunit 4",
  "gene": "UniProtKB:Q86V81",
  "gene_symbol": "ALYREF",
  "term_id": "GO:0003729",
  "term_label": "mRNA binding"
}